nuclear pore [GO:0005643] (cellular component) Sources: ISBN:0198547684 Also known as: NPC, nuclear pore complex, nucleopore, nuclear pore membrane protein Definition: A protein complex providing a discrete opening in the nuclear envelope of a eukaryotic cell, where the inner and outer nuclear membranes are joined. Relationships: is a type of nuclear protein-containing complex [GO:0140513]; is part of nuclear envelope [GO:0005635]